{
  "gene": "UniProtKB:Q05BU3",
  "term_label": "Unknown molecular function",
  "gene_symbol": "FAM86JP",
  "gene_name": "Putative protein FAM86JP",
  "term_id": "UNKNOWN:0001"
}